{
  "gene_symbol": "TMIGD3",
  "term_label": "immune response-activating signaling pathway",
  "term_id": "GO:0002757",
  "gene_name": "Transmembrane domain-containing protein TMIGD3",
  "gene": "UniProtKB:P0DMS9"
}